{
  "gene": "UniProtKB:Q9Y375",
  "gene_symbol": "NDUFAF1",
  "gene_name": "Complex I intermediate-associated protein 30, mitochondrial",
  "term_label": "unfolded protein binding",
  "term_id": "GO:0051082"
}